{
  "term_label": "cytoplasm",
  "gene_symbol": "CCNB1",
  "gene": "UniProtKB:P14635",
  "gene_name": "G2_mitotic-specific cyclin-B1",
  "term_id": "GO:0005737"
}